symbiont-mediated suppression of host transcription initiation from RNA polymerase II promoter [GO:0039602] (biological process) Definition: Any process in which a virus stops, prevents, or reduces the frequency, rate or extent of the assembly of the RNA polymerase II preinitiation complex (PIC) at an RNA polymerase II promoter region of a host DNA template. The host is defined as the larger of the organisms involved in a symbiotic interaction. References: PMID:1316611 Also known as: inhibition of host transcription initiation by virus, suppression by virus of host DNA-dependent transcription, initiation, suppression by virus of host transcription initiation from RNA polymerase II promoter Relationships: is a type of symbiont-mediated perturbation of host gene expression [GO:0039656]